positive regulation of leukocyte proliferation [GO:0070665] (biological process) Also known as: up regulation of leukocyte proliferation, up-regulation of leukocyte proliferation, upregulation of leukocyte proliferation, activation of leukocyte proliferation, stimulation of leukocyte proliferation Sources: GOC:add, GOC:mah Definition: Any process that activates or increases the frequency, rate or extent of leukocyte proliferation. Subtypes: positive regulation of mononuclear cell proliferation [GO:0032946], GO:0070668, GO:0090290, positive regulation of macrophage proliferation [GO:0120041] Relationships: is a type of positive regulation of cell population proliferation [GO:0008284]; is a type of regulation of leukocyte proliferation [GO:0070663]; positively regulates leukocyte proliferation [GO:0070661]